{
  "term_label": "extracellular matrix organization",
  "gene_symbol": "COL17A1",
  "gene": "UniProtKB:Q9UMD9",
  "term_id": "GO:0030198",
  "gene_name": "Collagen alpha-1(XVII) chain"
}